{
  "gene_symbol": "SMIM1",
  "gene_name": "Small integral membrane protein 1",
  "term_id": "UNKNOWN:0001",
  "term_label": "Unknown molecular function",
  "gene": "UniProtKB:B2RUZ4"
}